{
  "gene_symbol": "FAM74A7",
  "term_label": "Unknown molecular function",
  "gene": "UniProtKB:A6NL05",
  "term_id": "UNKNOWN:0001",
  "gene_name": "Protein FAM74A7"
}